pyrithiamine deaminase activity [GO:0050239] (molecular function) Also known as: 1-(4-amino-2-methylpyrimid-5-ylmethyl)-3-(beta-hydroxyethyl)-2-methylpyridinium-bromide aminohydrolase activity Definition: Catalysis of the reaction: 1-(4-amino-2-methylpyrimid-5-ylmethyl)-3-(beta-hydroxyethyl)-2-methylpyridinium bromide + H2O = 1-(4-hydroxy-2-methylpyrimid-5-ylmethyl)-3-(beta-hydroxyethyl)-2-methylpyridinium bromide + NH3. Sources: EC:3.5.4.20, MetaCyc:PYRITHIAMIN-DEAMINASE-RXN Relationships: is a type of hydrolase activity, acting on carbon-nitrogen (but not peptide) bonds, in cyclic amidines [GO:0016814]; is a type of deaminase activity [GO:0019239]